{
  "gene_symbol": "RASL11B",
  "term_label": "Unknown molecular function",
  "gene_name": "Ras-like protein family member 11B",
  "gene": "UniProtKB:Q9BPW5",
  "term_id": "UNKNOWN:0001"
}